{
  "gene": "UniProtKB:Q3SYC2",
  "term_id": "GO:0003846",
  "gene_name": "2-acylglycerol O-acyltransferase 2",
  "term_label": "2-acylglycerol O-acyltransferase activity",
  "gene_symbol": "MOGAT2"
}